regulation of type I interferon production [GO:0032479] (biological process) Relationships: is a type of regulation of cytokine production [GO:0001817]; regulates type I interferon production [GO:0032606] Definition: Any process that modulates the frequency, rate, or extent of interferon type I production. Type I interferons include the interferon-alpha, beta, delta, episilon, zeta, kappa, tau, and omega gene families. Subtypes: GO:0032480, positive regulation of type I interferon production [GO:0032481], regulation of interferon-alpha production [GO:0032647], GO:0032648 Sources: GOC:add, GOC:mah Also known as: regulation of type I IFN production